neuroepithelial cell differentiation [GO:0060563] (biological process) Regulation: negatively regulated by inhibition of neuroepithelial cell differentiation [GO:0002085]; positively regulated by positive regulation of neuroepithelial cell differentiation [GO:1902913] Sources: GOC:dph, GOC:tb Subtypes: GO:0061101, interstitial cell of Cajal differentiation [GO:0061453], GO:0071895 Definition: The process in which epiblast cells acquire specialized features of neuroepithelial cells. Relationships: is a type of GO:0002065